positive regulation of cAMP-dependent protein kinase activity [GO:2000481] (biological process) Definition: Any process that activates or increases the frequency, rate or extent of cAMP-dependent protein kinase activity. Sources: GOC:obol Also known as: positive regulation of 3',5' cAMP-dependent protein kinase activity, positive regulation of 3',5'-cAMP-dependent protein kinase activity, positive regulation of ATP:protein phosphotransferase (cAMP-dependent) activity, positive regulation of adenosine 3',5'-cyclophosphate-dependent protein kinase activity, positive regulation of cAMP-dependent protein kinase, intrinsic catalyst activity, positive regulation of cyclic AMP-dependent protein kinase activity, positive regulation of AMPK, positive regulation of PKA, positive regulation of PKA C, positive regulation of STK22, positive regulation of protein kinase A activity Relationships: is a type of positive regulation of protein serine/threonine kinase activity [GO:0071902]; is a type of GO:2000479; positively regulates GO:0004691